{
  "term_label": "adenylate cyclase-activating G protein-coupled receptor signaling pathway",
  "gene_symbol": "GLP1R",
  "gene": "UniProtKB:P43220",
  "term_id": "GO:0007189",
  "gene_name": "Glucagon-like peptide 1 receptor"
}